{
  "gene_symbol": "MCM5",
  "term_id": "GO:0042555",
  "gene": "UniProtKB:P33992",
  "term_label": "MCM complex",
  "gene_name": "DNA replication licensing factor MCM5"
}